Bolwig's organ morphogenesis [GO:0001746] (biological process) References: PMID:6185380 Definition: The morphogenetic process in which the anatomical structures of the larval eye in Drosophila are generated and organized. The larval eye in Drosophila is a relatively simple sensory system composed of Bolwig's organs: two clusters, each composed of 12 photoreceptor cells from which axons extend in a single fascicle to the brain. Relationships: is a type of eye morphogenesis [GO:0048592]; is part of GO:0055034